{
  "gene_name": "Immunoglobulin kappa variable 1_OR2-108 (non-functional) (Fragment)",
  "term_label": "Unknown molecular function",
  "gene_symbol": "IGKV1OR2-108",
  "term_id": "UNKNOWN:0001",
  "gene": "UniProtKB:A0A075B7D4"
}